diacylglyceride transfer activity [GO:0140337] (molecular function) Definition: Directly binding to diacylglyceride and delivering it either to an acceptor molecule or to a specific location. References: PMID:9132017 Also known as: diacylglyceride carrier activity Relationships: is a type of lipid transfer activity [GO:0120013]